{
  "term_id": "GO:0007156",
  "gene_name": "Pregnancy-specific beta-1-glycoprotein 5",
  "gene_symbol": "PSG5",
  "gene": "UniProtKB:Q15238",
  "term_label": "homophilic cell-cell adhesion"
}